{
  "gene_name": "Cyclic nucleotide-gated cation channel alpha-4",
  "gene": "UniProtKB:Q8IV77",
  "term_id": "GO:0017071",
  "term_label": "intracellular cyclic nucleotide activated cation channel complex",
  "gene_symbol": "CNGA4"
}